{
  "gene": "UniProtKB:P41143",
  "gene_symbol": "OPRD1",
  "term_label": "plasma membrane",
  "gene_name": "Delta-type opioid receptor",
  "term_id": "GO:0005886"
}